{
  "term_id": "GO:0000978",
  "gene_symbol": "ZNF648",
  "gene_name": "Zinc finger protein 648",
  "term_label": "RNA polymerase II cis-regulatory region sequence-specific DNA binding",
  "gene": "UniProtKB:Q5T619"
}